{
  "gene": "UniProtKB:P0DJ93",
  "term_label": "Unknown biological process",
  "gene_symbol": "SMIM13",
  "gene_name": "Small integral membrane protein 13",
  "term_id": "UNKNOWN:0002"
}